{
  "term_id": "GO:0031901",
  "term_label": "early endosome membrane",
  "gene_symbol": "SNX8",
  "gene_name": "Sorting nexin-8",
  "gene": "UniProtKB:Q9Y5X2"
}